{
  "gene_symbol": "LMLN",
  "gene_name": "Leishmanolysin-like peptidase",
  "term_id": "UNKNOWN:0002",
  "term_label": "Unknown biological process",
  "gene": "UniProtKB:Q96KR4"
}